{
  "gene_name": "Tetraspanin-13",
  "term_id": "UNKNOWN:0003",
  "term_label": "Unknown cellular component",
  "gene_symbol": "TSPAN13",
  "gene": "UniProtKB:O95857"
}